positive regulation of constitutive secretory pathway [GO:1903435] (biological process) Also known as: up regulation of constitutive secretory pathway, up-regulation of constitutive secretory pathway, upregulation of constitutive secretory pathway, activation of constitutive secretory pathway Definition: Any process that activates or increases the frequency, rate or extent of constitutive secretory pathway. References: PMID:22899725 Sources: GOC:TermGenie, GOC:als, GO_REF:0000058 Relationships: is a type of GO:0045921; is a type of regulation of constitutive secretory pathway [GO:1903433]; positively regulates GO:0045054